positive regulation of endothelial cell proliferation [GO:0001938] (biological process) Also known as: up regulation of endothelial cell proliferation, up-regulation of endothelial cell proliferation, upregulation of endothelial cell proliferation, activation of endothelial cell proliferation, stimulation of endothelial cell proliferation Definition: Any process that activates or increases the rate or extent of endothelial cell proliferation. Sources: GOC:add Relationships: is a type of regulation of endothelial cell proliferation [GO:0001936]; is a type of positive regulation of epithelial cell proliferation [GO:0050679]; RO_0002213 endothelial cell proliferation [GO:0001935] Subtypes: GO:1903589, positive regulation of vascular endothelial cell proliferation [GO:1905564]